{
  "gene": "UniProtKB:A6NMZ5",
  "gene_symbol": "OR4C45",
  "term_label": "olfactory receptor activity",
  "gene_name": "Olfactory receptor 4C45",
  "term_id": "GO:0004984"
}